{
  "gene": "UniProtKB:P49917",
  "term_label": "ATP binding",
  "gene_symbol": "LIG4",
  "term_id": "GO:0005524",
  "gene_name": "DNA ligase 4"
}